{
  "term_id": "GO:0006357",
  "gene_symbol": "ZNF880",
  "term_label": "regulation of transcription by RNA polymerase II",
  "gene_name": "Zinc finger protein 880",
  "gene": "UniProtKB:Q6PDB4"
}